negative regulation of miRNA metabolic process [GO:2000629] (biological process) Sources: GOC:dph Definition: Any process that stops, prevents or reduces the frequency, rate or extent of miRNA metabolic process. Also known as: negative regulation of microRNA metabolic process Relationships: is a type of negative regulation of RNA metabolic process [GO:0051253]; is a type of regulation of miRNA metabolic process [GO:2000628]; negatively regulates miRNA metabolic process [GO:0010586] Subtypes: negative regulation of miRNA transcription [GO:1902894], negative regulation of miRNA catabolic process [GO:2000626]